{
  "term_label": "Unknown molecular function",
  "gene_symbol": "PVALEF",
  "gene_name": "Parvalbumin-like EF-hand-containing protein",
  "term_id": "UNKNOWN:0001",
  "gene": "UniProtKB:A0A1B0GWK0"
}